regulation of cardiac vascular smooth muscle cell differentiation [GO:2000722] (biological process) Definition: Any process that modulates the frequency, rate or extent of cardiac vascular smooth muscle cell differentiation. Sources: GOC:BHF Subtypes: GO:2000723, GO:2000724 Relationships: is a type of GO:1905063; is a type of GO:1905207; regulates cardiac vascular smooth muscle cell differentiation [GO:0060947] Also known as: regulation of heart vascular smooth muscle cell differentiation